{
  "gene_name": "Pleckstrin homology domain-containing family M member 2",
  "term_id": "GO:0032418",
  "gene_symbol": "PLEKHM2",
  "gene": "UniProtKB:Q8IWE5",
  "term_label": "lysosome localization"
}